synaptonemal complex disassembly [GO:0070194] (biological process) Definition: The controlled breakdown of a synaptonemal complex. Relationships: is_a cellular component disassembly [GO:0022411]; is a type of synaptonemal complex organization [GO:0070193] Sources: GOC:mah